{
  "term_id": "UNKNOWN:0001",
  "term_label": "Unknown molecular function",
  "gene_symbol": "Q6ZVH6",
  "gene": "UniProtKB:Q6ZVH6",
  "gene_name": "Putative uncharacterized protein FLJ42569"
}